trans-epoxysuccinate hydrolase activity [GO:0050345] (molecular function) Also known as: tartrate epoxydase activity, trans-2,3-epoxysuccinate hydrolase activity, trans-epoxysuccinate hydratase activity Sources: EC:3.3.2.4, RHEA:20740 Definition: Catalysis of the reaction: trans-2,3-epoxysuccinate + H2O = (2R,3S)-tartrate. Relationships: is a type of GO:0016803